positive regulation of spindle assembly [GO:1905832] (biological process) Relationships: is a type of positive regulation of cytoskeleton organization [GO:0051495]; is a type of positive regulation of cell cycle process [GO:0090068]; is a type of GO:0090169; is_a positive regulation of organelle assembly [GO:1902117]; positively regulates spindle assembly [GO:0051225] Definition: Any process that activates or increases the frequency, rate or extent of spindle assembly. References: PMID:27689799 Sources: GOC:TermGenie, GO_REF:0000058 Also known as: positive regulation of bipolar spindle biosynthesis, positive regulation of bipolar spindle formation, positive regulation of spindle biosynthesis, positive regulation of spindle formation, up regulation of bipolar spindle biosynthesis, up regulation of bipolar spindle formation, up regulation of spindle assembly, up regulation of spindle biosynthesis, up regulation of spindle formation, up-regulation of bipolar spindle biosynthesis, up-regulation of bipolar spindle formation, up-regulation of spindle assembly, up-regulation of spindle biosynthesis, up-regulation of spindle formation, upregulation of bipolar spindle biosynthesis, upregulation of bipolar spindle formation, upregulation of spindle assembly, upregulation of spindle biosynthesis, upregulation of spindle formation, activation of bipolar spindle biosynthesis, activation of bipolar spindle formation, activation of spindle assembly, activation of spindle biosynthesis, activation of spindle formation Subtypes: GO:0110161